{
  "gene_symbol": "XRN2",
  "term_id": "GO:0004534",
  "gene": "UniProtKB:Q9H0D6",
  "term_label": "5'-3' RNA exonuclease activity",
  "gene_name": "5'-3' exoribonuclease 2"
}